natural killer cell degranulation [GO:0043320] (biological process) Regulation: RO_0002211 by regulation of natural killer cell degranulation [GO:0043321]; negatively regulated by negative regulation of natural killer cell degranulation [GO:0043322]; positively regulated by positive regulation of natural killer cell degranulation [GO:0043323] Relationships: is a type of leukocyte degranulation [GO:0043299]; is part of natural killer cell activation involved in immune response [GO:0002323]; is part of natural killer cell mediated cytotoxicity [GO:0042267] Definition: The regulated exocytosis of secretory granules containing preformed mediators such as perforin and granzymes by a natural killer cell. Sources: ISBN:0781735149 Also known as: NK cell degranulation, NK cell granule exocytosis, natural killer cell granule exocytosis